{
  "gene_name": "ATP-dependent RNA helicase TDRD9",
  "term_id": "UNKNOWN:0002",
  "gene": "UniProtKB:Q8NDG6",
  "gene_symbol": "TDRD9",
  "term_label": "Unknown biological process"
}